{
  "term_id": "UNKNOWN:0002",
  "gene_symbol": "DNAJC9-AS1",
  "gene": "UniProtKB:A6NH13",
  "gene_name": "Putative uncharacterized protein DNAJC9-AS1",
  "term_label": "Unknown biological process"
}